{
  "gene": "UniProtKB:Q07817",
  "gene_symbol": "BCL2L1",
  "term_id": "GO:0008630",
  "term_label": "intrinsic apoptotic signaling pathway in response to DNA damage",
  "gene_name": "Bcl-2-like protein 1"
}